{
  "term_id": "GO:0004843",
  "gene": "UniProtKB:Q9BXU7",
  "gene_name": "Ubiquitin carboxyl-terminal hydrolase 26",
  "gene_symbol": "USP26",
  "term_label": "cysteine-type deubiquitinase activity"
}